brexanolone metabolic process [GO:0062173] (biological process) Relationships: is a type of steroid metabolic process [GO:0008202]; is a type of ketone metabolic process [GO:0042180] Subtypes: GO:0062174, brexanolone catabolic process [GO:0062175] Definition: The chemical reactions and pathways by which living organisms transform brexanolone. References: PMID:24390875 Also known as: allopregnanolone metabolic process, allopregnanolone metabolism, allotetrahydroprogesterone metabolic process, allotetrahydroprogesterone metabolism, brexanolone metabolism